{
  "gene_name": "BTB_POZ domain-containing protein KCTD17",
  "gene_symbol": "KCTD17",
  "term_id": "GO:0097602",
  "term_label": "cullin family protein binding",
  "gene": "UniProtKB:Q8N5Z5"
}